{
  "gene_name": "WD repeat-containing protein 6",
  "gene_symbol": "WDR6",
  "term_id": "GO:0005737",
  "term_label": "cytoplasm",
  "gene": "UniProtKB:Q9NNW5"
}